{
  "gene_symbol": "PCID2",
  "gene_name": "PCI domain-containing protein 2",
  "term_label": "transcription export complex 2",
  "term_id": "GO:0070390",
  "gene": "UniProtKB:Q5JVF3"
}